{
  "term_id": "GO:0004016",
  "term_label": "adenylate cyclase activity",
  "gene_symbol": "ADCY3",
  "gene_name": "Adenylate cyclase type 3",
  "gene": "UniProtKB:O60266"
}